{
  "term_label": "retrograde transport, endosome to Golgi",
  "gene_name": "WASH complex subunit 1",
  "gene_symbol": "WASHC1",
  "gene": "UniProtKB:A8K0Z3",
  "term_id": "GO:0042147"
}